raucaffricine beta-glucosidase activity [GO:0050247] (molecular function) Definition: Catalysis of the reaction: H2O + raucaffricine = D-glucose + vomilenine. Sources: EC:3.2.1.125, RHEA:14557 Relationships: is a type of beta-glucosidase activity [GO:0008422] Also known as: raucaffricine b-glucosidase activity, raucaffricine beta-D-glucohydrolase activity, raucaffricine beta-D-glucosidase activity, raucaffricine glucosidase activity